5-diphosphoinositol pentakisphosphate 4-kinase activity [GO:0000833] (molecular function) Definition: Catalysis of the reaction: ATP + 5-diphospho-1D-myo-inositol (1,2,3,4,6)pentakisphosphate = ADP + 4,5-bis(diphospho)-1D-myo-inositol (1,2,3,6)tetrakisphosphate. References: PMID:16429326 Sources: GOC:elh Also known as: diphosphoinositol-pentakisphosphate 4-kinase activity, inositol heptakisphosphate 4-kinase activity, IP7 4-kinase activity Relationships: is_a diphosphoinositol pentakisphosphate kinase activity [GO:0000829]